genital disc anterior/posterior pattern formation [GO:0035224] (biological process) Relationships: is a type of GO:0007448; is a type of genital disc pattern formation [GO:0035221] Definition: The establishment, maintenance and elaboration of the anterior/posterior axis of the genital disc. An anterior and posterior compartment form in each of the three genital disc primoridia (the female genital disc primordium, the male genital disc primordium and the anal primordium). References: PMID:11494318